{
  "term_id": "GO:0007010",
  "gene_name": "PH-interacting protein",
  "term_label": "cytoskeleton organization",
  "gene_symbol": "PHIP",
  "gene": "UniProtKB:Q8WWQ0"
}